{
  "term_label": "negative regulation of ERK1 and ERK2 cascade",
  "gene_symbol": "SPRY1",
  "gene": "UniProtKB:O43609",
  "term_id": "GO:0070373",
  "gene_name": "Protein sprouty homolog 1"
}